ferredoxin-nitrite reductase activity [GO:0048307] (molecular function) Relationships: is_a oxidoreductase activity, acting on other nitrogenous compounds as donors, iron-sulfur protein as acceptor [GO:0016664]; is a type of nitrite reductase activity [GO:0098809] Definition: Catalysis of the reaction: 2 H2O + NH4+ + 6 oxidized [2Fe-2S]-[ferredoxin] = 8 H+ + nitrite + 6 reduced [2Fe-2S]-[ferredoxin]. Also known as: ammonia:ferredoxin oxidoreductase activity Sources: RHEA:18041